{
  "gene": "UniProtKB:O00116",
  "term_id": "GO:0005777",
  "gene_name": "Alkyldihydroxyacetonephosphate synthase, peroxisomal",
  "term_label": "peroxisome",
  "gene_symbol": "AGPS"
}